{
  "gene_symbol": "TAF11L14",
  "gene_name": "TATA-box-binding protein-associated factor 11-like protein 14",
  "term_id": "GO:0051123",
  "gene": "UniProtKB:A0A1W2PPL8",
  "term_label": "RNA polymerase II preinitiation complex assembly"
}